{
  "gene_symbol": "NLRP12",
  "gene_name": "NACHT, LRR and PYD domains-containing protein 12",
  "gene": "UniProtKB:P59046",
  "term_id": "GO:1901223",
  "term_label": "negative regulation of non-canonical NF-kappaB signal transduction"
}